{
  "gene_name": "Metallothionein-1E",
  "gene": "UniProtKB:P04732",
  "term_label": "intracellular zinc ion homeostasis",
  "term_id": "GO:0006882",
  "gene_symbol": "MT1E"
}